{
  "term_label": "base-excision repair",
  "term_id": "GO:0006284",
  "gene": "UniProtKB:P27695",
  "gene_name": "DNA-(apurinic or apyrimidinic site) endonuclease",
  "gene_symbol": "APEX1"
}